{
  "term_label": "response to nutrient levels",
  "gene": "UniProtKB:P01242",
  "gene_name": "Growth hormone variant",
  "term_id": "GO:0031667",
  "gene_symbol": "GH2"
}